{
  "term_id": "GO:0005737",
  "gene_symbol": "PI4KB",
  "gene": "UniProtKB:Q9UBF8",
  "term_label": "cytoplasm",
  "gene_name": "Phosphatidylinositol 4-kinase beta"
}